{
  "term_label": "Unknown biological process",
  "term_id": "UNKNOWN:0002",
  "gene_name": "NAD(+) hydrolase SARM1",
  "gene_symbol": "SARM1",
  "gene": "UniProtKB:Q6SZW1"
}